{
  "gene_symbol": "ZSCAN18",
  "term_label": "Unknown cellular component",
  "term_id": "UNKNOWN:0003",
  "gene_name": "Zinc finger and SCAN domain-containing protein 18",
  "gene": "UniProtKB:Q8TBC5"
}